{
  "gene": "UniProtKB:Q8IUG5",
  "term_id": "GO:0051015",
  "gene_name": "Unconventional myosin-XVIIIb",
  "gene_symbol": "MYO18B",
  "term_label": "actin filament binding"
}